{
  "term_id": "UNKNOWN:0002",
  "gene": "UniProtKB:Q8NGJ0",
  "gene_symbol": "OR5A1",
  "term_label": "Unknown biological process",
  "gene_name": "Olfactory receptor 5A1"
}